{
  "term_id": "GO:0006164",
  "gene_name": "Ribose-phosphate pyrophosphokinase 1",
  "gene_symbol": "PRPS1",
  "gene": "UniProtKB:P60891",
  "term_label": "purine nucleotide biosynthetic process"
}